{
  "term_id": "GO:0042867",
  "gene_name": "L-lactate dehydrogenase A chain",
  "gene": "UniProtKB:P00338",
  "term_label": "pyruvate catabolic process",
  "gene_symbol": "LDHA"
}